karyogamy [GO:0000741] (biological process) Also known as: nuclear fusion, nuclear fusion during karyogamy Subtypes: GO:0000742, karyogamy involved in conjugation with mutual genetic exchange [GO:0000744], pronuclear fusion [GO:0007344], polar nucleus fusion [GO:0010197] Relationships: is a type of nucleus organization [GO:0006997]; is a type of GO:0048284; is part of nucleus organization [GO:0006997] Sources: GOC:elh Definition: The creation of a single nucleus from multiple nuclei as a result of fusing the lipid bilayers that surround each nuclei. Regulation: regulated by regulation of karyogamy [GO:0032871]